{
  "gene_name": "GATOR complex protein WDR59",
  "term_label": "Seh1-associated complex",
  "term_id": "GO:0035859",
  "gene": "UniProtKB:Q6PJI9",
  "gene_symbol": "WDR59"
}